coumarin catabolic process [GO:0046226] (biological process) Relationships: is a type of coumarin metabolic process [GO:0009804]; is a type of phenylpropanoid catabolic process [GO:0046271] Sources: GOC:ai Also known as: coumarin breakdown, coumarin catabolism, coumarin degradation Definition: The chemical reactions and pathways resulting in the breakdown of coumarins, compounds derived from the phenylacrylic skeleton of cinnamic acids. Subtypes: GO:1901883